dihydroxy-acid dehydratase activity [GO:0004160] (molecular function) Definition: Catalysis of the reaction: (2R)-2,3-dihydroxy-3-methylbutanoate = 3-methyl-2-oxobutanoate + H2O. Also known as: 2,3-dihydroxy-acid hydro-lyase (3-methyl-2-oxobutanoate-forming), 2,3-dihydroxy-acid hydro-lyase activity, 2,3-dihydroxyisovalerate dehydratase activity, DHAD, acetohydroxyacid dehydratase activity, alpha,beta-dihydroxyacid dehydratase activity, alpha,beta-dihydroxyisovalerate dehydratase activity, dihydroxy acid dehydrase activity Sources: RHEA:24809 Relationships: is a type of GO:0016836